potassium ion uniporter activity [GO:0022819] (molecular function) Sources: GOC:mtg_transport, ISBN:0815340729 Relationships: is a type of potassium ion transmembrane transporter activity [GO:0015079]; is a type of membrane potential driven uniporter activity [GO:0022810] Definition: Catalysis of the active transport of a potassium ion across a membrane by a mechanism involving conformational change, where energy for active transport is derived from membrane potential if the solute is charged.